thiosulfate-cyanide sulfurtransferase activity [GO:0004792] (molecular function) Also known as: thiosulfate sulfurtransferase activity, thiosulphate sulphurtransferase activity, rhodanase activity, rhodanese activity, thiosulfate cyanide transsulfurase activity, thiosulfate thiotransferase activity, thiosulfate:cyanide sulfurtransferase activity Sources: RHEA:16881 Definition: Catalysis of the reaction: thiosulfate + hydrogen cyanide = thiocyanate + sulfite + 2 H+. Relationships: is a type of sulfurtransferase activity [GO:0016783]